{
  "gene_symbol": "GCG",
  "gene_name": "Pro-glucagon",
  "gene": "UniProtKB:P01275",
  "term_label": "extracellular space",
  "term_id": "GO:0005615"
}